negative regulation of Notch signaling pathway [GO:0045746] (biological process) Relationships: is a type of regulation of Notch signaling pathway [GO:0008593]; is a type of negative regulation of signal transduction [GO:0009968]; RO_0002212 Notch signaling pathway [GO:0007219] Subtypes: negative regulation of Notch signaling pathway involved in somitogenesis [GO:1902367] Sources: GOC:go_curators Also known as: down regulation of Notch signaling pathway, down-regulation of Notch signaling pathway, downregulation of Notch signaling pathway, negative regulation of N signaling pathway, negative regulation of N signalling pathway, negative regulation of Notch signalling pathway, inhibition of Notch signaling pathway Definition: Any process that stops, prevents, or reduces the frequency, rate or extent of the Notch signaling pathway.